{
  "gene_name": "SERTA domain-containing protein 1",
  "gene_symbol": "SERTAD1",
  "term_label": "cytoplasm",
  "term_id": "GO:0005737",
  "gene": "UniProtKB:Q9UHV2"
}